gluconate transmembrane transport [GO:0035429] (biological process) Definition: The process in which gluconate is transported across a membrane. Gluconate is the aldonic acid derived from glucose. Sources: GOC:vw, ISBN:0198506732 Also known as: gluconate membrane transport, gluconate transport Note: Note that this term is not intended for use in annotating lateral movement within membranes. Relationships: is_a aldonate transmembrane transport [GO:0042873] Subtypes: gluconate import across plasma membrane [GO:0140270] Regulation: regulated by regulation of gluconate transmembrane transport [GO:0035430]; negatively regulated by negative regulation of gluconate transmembrane transport [GO:0035431]; positively regulated by positive regulation of gluconate transmembrane transport [GO:0035432]